{
  "gene_name": "N-alpha-acetyltransferase 40",
  "term_id": "GO:0005634",
  "gene_symbol": "NAA40",
  "gene": "UniProtKB:Q86UY6",
  "term_label": "nucleus"
}